VEGF-A complex [GO:1990150] (cellular component) Definition: A homodimeric, extracellular protein complex containing two VEGF-A monomers. Binds to and activates a receptor tyrosine kinase. Also known as: vascular endothelial growth factor A complex Relationships: is_a growth factor complex [GO:0036454] References: PMID:12207021, PMID:19658168 Sources: GOC:bf, GOC:bhm